butanol dehydrogenase (NAD+) activity [GO:1990362] (molecular function) Definition: Catalysis of the reaction: butan-1-ol + NAD+ = butanal + H+ + NADH. Also known as: butanol dehydrogenase activity Relationships: is a type of alcohol dehydrogenase (NAD+) activity [GO:0004022] References: PMID:1999395 Sources: GOC:mengo_curators, RHEA:33199